{
  "term_id": "GO:0004090",
  "gene_name": "Dehydrogenase_reductase SDR family member 4-like 2",
  "term_label": "carbonyl reductase (NADPH) activity",
  "gene_symbol": "DHRS4L2",
  "gene": "UniProtKB:Q6PKH6"
}